{
  "gene_symbol": "CHRNE",
  "gene": "UniProtKB:Q04844",
  "term_label": "acetylcholine-gated monoatomic cation-selective channel activity",
  "gene_name": "Acetylcholine receptor subunit epsilon",
  "term_id": "GO:0022848"
}